{
  "gene_name": "Metallothionein-1E",
  "gene": "UniProtKB:P04732",
  "term_id": "GO:0005737",
  "gene_symbol": "MT1E",
  "term_label": "cytoplasm"
}